{
  "gene_symbol": "FSTL5",
  "gene": "UniProtKB:Q8N475",
  "term_id": "GO:0030154",
  "term_label": "cell differentiation",
  "gene_name": "Follistatin-related protein 5"
}